{
  "term_label": "heterotrimeric G-protein complex assembly",
  "term_id": "GO:1902605",
  "gene": "UniProtKB:Q13371",
  "gene_name": "Phosducin-like protein",
  "gene_symbol": "PDCL"
}